{
  "gene_symbol": "PPM1N",
  "term_label": "cytosol",
  "gene_name": "Probable protein phosphatase 1N",
  "gene": "UniProtKB:Q8N819",
  "term_id": "GO:0005829"
}